{
  "gene_name": "Advanced glycosylation end product-specific receptor",
  "term_label": "microglial cell activation",
  "gene_symbol": "AGER",
  "term_id": "GO:0001774",
  "gene": "UniProtKB:Q15109"
}